nitrogenase P cluster assembly [GO:0044573] (biological process) Also known as: nitrogenase P cluster biosynthesis, nitrogenase P cluster maturation References: PMID:17563349 Definition: The biochemical reactions and pathways resulting in the formation of a P-cluster of a nitrogenase, a high-nuclearity, Fe/S-only cluster that can be viewed as two [4Fe-4S] sub-clusters sharing a gamma-6-sulfide. Relationships: is_a iron-sulfur cluster assembly [GO:0016226]